{
  "gene": "UniProtKB:Q13557",
  "term_id": "GO:0005516",
  "term_label": "calmodulin binding",
  "gene_symbol": "CAMK2D",
  "gene_name": "Calcium_calmodulin-dependent protein kinase type II subunit delta"
}